{
  "gene_symbol": "IGKV3D-7",
  "term_label": "immune response",
  "gene": "UniProtKB:A0A0C4DH55",
  "term_id": "GO:0006955",
  "gene_name": "Immunoglobulin kappa variable 3D-7"
}